{
  "gene": "UniProtKB:Q9ULV1",
  "term_id": "GO:0042813",
  "gene_symbol": "FZD4",
  "gene_name": "Frizzled-4",
  "term_label": "Wnt receptor activity"
}